lipoamidase activity [GO:0061690] (molecular function) Definition: Catalysis of the reaction: H2O + N(6)-[(R)-lipoyl]-L-lysyl-[lipoyl-carrier protein] = (R)-lipoate + L-lysyl-[lipoyl-carrier protein]. References: PMID:14086741 Sources: RHEA:76519 Relationships: is a type of GO:0016811 Also known as: lipoyl-X-hydrolase